{
  "gene": "UniProtKB:P49585",
  "gene_symbol": "PCYT1A",
  "gene_name": "Choline-phosphate cytidylyltransferase A",
  "term_label": "Unknown biological process",
  "term_id": "UNKNOWN:0002"
}